neutral lipid biosynthetic process [GO:0046460] (biological process) Also known as: neutral lipid anabolism, neutral lipid biosynthesis, neutral lipid formation, neutral lipid synthesis Sources: GOC:ai Relationships: is a type of neutral lipid metabolic process [GO:0006638]; is a type of GO:0008610 Definition: The chemical reactions and pathways resulting in the formation of neutral lipids, lipids only soluble in solvents of very low polarity. Subtypes: acylglycerol biosynthetic process [GO:0046463]